glucose-fructose oxidoreductase activity [GO:0047061] (molecular function) Definition: Catalysis of the reaction: D-fructose + D-glucose = D-glucitol + D-glucono-1,5-lactone. Sources: EC:1.1.99.28, RHEA:20637 Also known as: D-glucose:D-fructose oxidoreductase activity Relationships: is a type of oxidoreductase activity, acting on CH-OH group of donors [GO:0016614]